{
  "term_label": "integrin alphaX-beta2 complex",
  "term_id": "GO:0034689",
  "gene_symbol": "ITGAX",
  "gene": "UniProtKB:P20702",
  "gene_name": "Integrin alpha-X"
}